{
  "gene_name": "Metastasis-associated protein MTA2",
  "gene_symbol": "MTA2",
  "term_id": "GO:0042826",
  "term_label": "histone deacetylase binding",
  "gene": "UniProtKB:O94776"
}